{
  "term_id": "GO:0022625",
  "gene_name": "Ribosomal protein eL39-like 2",
  "gene_symbol": "RPL39L",
  "gene": "UniProtKB:Q96EH5",
  "term_label": "cytosolic large ribosomal subunit"
}